{
  "term_id": "GO:0007165",
  "gene": "UniProtKB:Q6UX06",
  "term_label": "signal transduction",
  "gene_symbol": "OLFM4",
  "gene_name": "Olfactomedin-4"
}